{
  "term_label": "immune response",
  "term_id": "GO:0006955",
  "gene": "UniProtKB:A0A1B0GX56",
  "gene_symbol": "TRDV1",
  "gene_name": "T cell receptor delta variable 1"
}